{
  "gene_name": "Cadherin-related family member 5",
  "term_label": "cell adhesion molecule binding",
  "term_id": "GO:0050839",
  "gene": "UniProtKB:Q9HBB8",
  "gene_symbol": "CDHR5"
}